methylamine-glutamate N-methyltransferase activity [GO:0047148] (molecular function) Definition: Catalysis of the reaction: L-glutamate + methylammonium = N-methyl-L-glutamate + NH4. Also known as: N-methylglutamate synthase activity, methylamine-glutamate methyltransferase activity, methylamine:L-glutamate N-methyltransferase activity Relationships: is a type of GO:0008170 Sources: EC:2.1.1.21, RHEA:15837